{
  "gene": "UniProtKB:Q9NPI8",
  "term_id": "GO:0043240",
  "term_label": "Fanconi anaemia nuclear complex",
  "gene_symbol": "FANCF",
  "gene_name": "Fanconi anemia group F protein"
}